{
  "gene": "UniProtKB:Q9Y4G6",
  "gene_name": "Talin-2",
  "gene_symbol": "TLN2",
  "term_label": "cell-cell adhesion",
  "term_id": "GO:0098609"
}